urotensin receptor binding [GO:0031889] (molecular function) Also known as: urotensin receptor ligand Definition: Binding to a urotensin receptor. Relationships: is a type of G protein-coupled receptor binding [GO:0001664] Sources: GOC:mah, GOC:nln